{
  "gene_symbol": "TUBG2",
  "term_label": "meiotic spindle organization",
  "gene_name": "Tubulin gamma-2 chain",
  "term_id": "GO:0000212",
  "gene": "UniProtKB:Q9NRH3"
}